isocitrate metabolic process [GO:0006102] (BP) Definition: The chemical reactions and pathways involving isocitrate, the anion of isocitric acid, 1-hydroxy-1,2,3-propanetricarboxylic acid. Isocitrate is an important intermediate in the TCA cycle and the glycoxylate cycle. Sources: ISBN:0198506732 Also known as: isocitrate metabolism Relationships: is a type of tricarboxylic acid metabolic process [GO:0072350]; is a type of secondary alcohol metabolic process [GO:1902652]